{
  "gene_name": "Immunoglobulin heavy variable 1-8",
  "term_label": "immunoglobulin mediated immune response",
  "gene_symbol": "IGHV1-8",
  "term_id": "GO:0016064",
  "gene": "UniProtKB:P0DP01"
}